trans-translation-dependent protein tagging [GO:0070930] (biological process) References: PMID:11395451, PMID:35264790 Also known as: co-translational protein tagging, cotranslational protein tagging, protein modification by trans-translation Relationships: is a type of rescue of stalled ribosome [GO:0072344]; has part trans-translation [GO:0070929] Note: Note that this term is not a child of 'co-translational protein modification process ; GO:0043686' because co-translational protein modification implies modification of a previously incorporated amino acid in a nascent chain, rather than addition of new sequence to the C-terminus. Definition: A protein modification process in which a polypeptide is added to a nascent polypeptide cotranslationally by trans-translation.